{
  "gene_name": "Serine palmitoyltransferase 2",
  "gene_symbol": "SPTLC2",
  "term_id": "GO:0017059",
  "gene": "UniProtKB:O15270",
  "term_label": "serine palmitoyltransferase complex"
}